positive regulation of T cell cytokine production [GO:0002726] (biological process) Sources: GOC:add Relationships: is a type of positive regulation of T cell mediated immunity [GO:0002711]; is a type of positive regulation of cytokine production involved in immune response [GO:0002720]; is a type of GO:0002724; RO_0002213 T cell cytokine production [GO:0002369] Subtypes: positive regulation of T-helper 2 cell cytokine production [GO:2000553], positive regulation of T-helper 1 cell cytokine production [GO:2000556] Also known as: positive regulation of T lymphocyte cytokine production, positive regulation of T-cell cytokine production, positive regulation of T-lymphocyte cytokine production, up regulation of T cell cytokine production, up-regulation of T cell cytokine production, upregulation of T cell cytokine production, activation of T cell cytokine production, stimulation of T cell cytokine production Definition: Any process that activates or increases the frequency, rate, or extent of T cell cytokine production.